{
  "gene_name": "Centrosomal protein of 135 kDa",
  "gene": "UniProtKB:Q66GS9",
  "term_id": "UNKNOWN:0001",
  "gene_symbol": "CEP135",
  "term_label": "Unknown molecular function"
}